urea metabolic process [GO:0019627] (biological process) Definition: The chemical reactions and pathways involving urea, the water soluble compound O=C-(NH2)2. Sources: ISBN:0198506732 Also known as: urea metabolism Relationships: is a type of GO:0043603; is a type of GO:0044281; is a type of nitrogen cycle metabolic process [GO:0071941] Subtypes: GO:0000050, atrazine catabolic process to urea [GO:0019623], urea catabolic process [GO:0043419]